{
  "term_label": "Unknown molecular function",
  "gene_name": "Small cysteine and glycine repeat-containing protein 9",
  "term_id": "UNKNOWN:0001",
  "gene": "UniProtKB:P0DSO2",
  "gene_symbol": "SCYGR9"
}